formation of animal organ boundary [GO:0010160] (biological process) Also known as: organ boundary specification References: PMID:9611175 Sources: GOC:dph, GOC:isa_complete Relationships: is a type of regionalization [GO:0003002]; is a type of formation of anatomical boundary [GO:0048859]; is part of GO:0048645 Subtypes: salivary gland boundary specification [GO:0007432], sensory organ boundary specification [GO:0008052] Definition: The regionalization process that specifies animal organ primordium boundaries resulting in a restriction of organogenesis to a limited spatial domain and keeping the organ separate from surrounding tissues.